{
  "gene_symbol": "DTX3",
  "term_label": "nucleoplasm",
  "gene_name": "Probable E3 ubiquitin-protein ligase DTX3",
  "term_id": "GO:0005654",
  "gene": "UniProtKB:Q8N9I9"
}